{
  "gene_symbol": "SPATA31C2",
  "term_label": "Unknown molecular function",
  "gene_name": "Putative spermatogenesis-associated protein 31C2",
  "term_id": "UNKNOWN:0001",
  "gene": "UniProtKB:B4DYI2"
}